{
  "gene_symbol": "DKFZp781C0719",
  "gene": "UniProtKB:Q68DW6",
  "term_label": "Unknown biological process",
  "gene_name": "Uncharacterized protein DKFZp781C0719",
  "term_id": "UNKNOWN:0002"
}